{
  "gene_name": "Myosin-binding protein H-like",
  "gene_symbol": "MYBPHL",
  "term_label": "Unknown molecular function",
  "term_id": "UNKNOWN:0001",
  "gene": "UniProtKB:A2RUH7"
}